{
  "term_label": "regulation of transcription by RNA polymerase II",
  "gene_symbol": "ZNF543",
  "term_id": "GO:0006357",
  "gene": "UniProtKB:Q08ER8",
  "gene_name": "Zinc finger protein 543"
}